{
  "term_label": "meiotic DNA double-strand break formation",
  "gene": "UniProtKB:Q9Y5K1",
  "gene_name": "Meiotic recombination protein SPO11",
  "gene_symbol": "SPO11",
  "term_id": "GO:0042138"
}